{
  "gene_name": "Ubiquinol-cytochrome-c reductase complex assembly factor 2",
  "term_label": "mitochondrial respiratory chain complex III assembly",
  "gene_symbol": "UQCC2",
  "term_id": "GO:0034551",
  "gene": "UniProtKB:Q9BRT2"
}